{
  "gene": "UniProtKB:A2VDJ0",
  "term_id": "GO:0005886",
  "gene_symbol": "TMEM131L",
  "gene_name": "Transmembrane protein 131-like",
  "term_label": "plasma membrane"
}